{
  "gene": "UniProtKB:Q9Y6C5",
  "gene_name": "Protein patched homolog 2",
  "term_id": "GO:0008158",
  "term_label": "hedgehog receptor activity",
  "gene_symbol": "PTCH2"
}